{
  "gene_symbol": "METTL4",
  "gene": "UniProtKB:Q8N3J2",
  "term_label": "Unknown biological process",
  "gene_name": "N(6)-adenine-specific methyltransferase METTL4",
  "term_id": "UNKNOWN:0002"
}